dorsal motor nucleus of vagus nerve structural organization [GO:0035763] (biological process) Definition: The process that contributes to the act of creating the structural organization of the dorsal motor nucleus of the vagus nerve. This process pertains to the physical shaping of a rudimentary structure. Relationships: is a type of GO:0048532; is part of dorsal motor nucleus of vagus nerve morphogenesis [GO:0035762] Also known as: dorsal motor nucleus of vagus nerve structural organisation Sources: GOC:dgh